{
  "gene": "UniProtKB:A0A6Q8PHR7",
  "term_label": "Unknown molecular function",
  "term_id": "UNKNOWN:0001",
  "gene_name": "Uncharacterized protein",
  "gene_symbol": "A0A6Q8PHR7"
}